{
  "gene": "UniProtKB:Q8WU20",
  "term_label": "transmembrane receptor protein tyrosine kinase adaptor activity",
  "gene_name": "Fibroblast growth factor receptor substrate 2",
  "term_id": "GO:0005068",
  "gene_symbol": "FRS2"
}